mitochondrial permeability transition pore complex [GO:0005757] (cellular component) Also known as: PTPC, MPTP complex, mitochondrial PT pore complex Relationships: is a type of pore complex [GO:0046930]; is a type of GO:0098798; is part of mitochondrial envelope [GO:0005740] References: PMID:10393078 Definition: A protein complex that connects the inner and outer membranes of animal mitochondria and acts as a pore that can open transiently to allow free diffusion of solutes between the mitochondrial matrix and the cytosol. The pore complex is formed of the voltage-dependent anion channel (VDAC), the adenine nucleotide translocase (ANT) and cyclophilin-D (CyP-D).